{
  "term_id": "GO:0005615",
  "gene": "UniProtKB:Q5T4F7",
  "gene_symbol": "SFRP5",
  "term_label": "extracellular space",
  "gene_name": "Secreted frizzled-related protein 5"
}